{
  "gene": "UniProtKB:O95619",
  "gene_name": "YEATS domain-containing protein 4",
  "gene_symbol": "YEATS4",
  "term_label": "regulation of transcription by RNA polymerase II",
  "term_id": "GO:0006357"
}